{
  "gene": "UniProtKB:Q9H4G0",
  "gene_name": "Band 4.1-like protein 1",
  "term_id": "GO:0005856",
  "term_label": "cytoskeleton",
  "gene_symbol": "EPB41L1"
}